{
  "gene": "UniProtKB:Q13422",
  "gene_name": "DNA-binding protein Ikaros",
  "term_id": "GO:0000978",
  "term_label": "RNA polymerase II cis-regulatory region sequence-specific DNA binding",
  "gene_symbol": "IKZF1"
}